cell chemotaxis to vascular endothelial growth factor [GO:0090667] (biological process) Relationships: is a type of cell chemotaxis [GO:0060326]; is part of GO:0035924 Definition: The directed movement of a motile cell in response to the presence of vascular endothelial growth factor (VEGF). References: PMID:21885851 Sources: GOC:BHF, GOC:BHF_miRNA, GOC:rph Subtypes: endothelial cell chemotaxis to vascular endothelial growth factor [GO:0090668]